{
  "term_label": "nitric oxide mediated signal transduction",
  "gene_symbol": "NOS1",
  "gene_name": "Nitric oxide synthase 1",
  "term_id": "GO:0007263",
  "gene": "UniProtKB:P29475"
}